nicotinamide nucleotide biosynthetic process [GO:0019359] (biological process) Subtypes: NADP+ biosynthetic process [GO:0006741], NAD+ biosynthetic process [GO:0009435], nicotinamide nucleotide biosynthetic process from niacinamide [GO:0019360] Relationships: is a type of pyridine nucleotide biosynthetic process [GO:0019363]; is a type of GO:0046496 Sources: GOC:go_curators Definition: The chemical reactions and pathways resulting in the formation of nicotinamide nucleotides, any nucleotide that contains combined nicotinamide. Also known as: nicotinamide nucleotide anabolism, nicotinamide nucleotide biosynthesis, nicotinamide nucleotide formation, nicotinamide nucleotide synthesis